imaginal disc pattern formation [GO:0007447] (biological process) Relationships: is a type of GO:0003002; is part of imaginal disc development [GO:0007444] Subtypes: anterior/posterior pattern specification, imaginal disc [GO:0007448], proximal/distal pattern formation, imaginal disc [GO:0007449], dorsal/ventral pattern formation, imaginal disc [GO:0007450], genital disc pattern formation [GO:0035221], GO:0035222, leg disc pattern formation [GO:0035223] Definition: The regionalization process that results in defined areas of the imaginal disc that will undergo specific cell differentaiton. Imaginal discs are epithelial infoldings in the larvae of holometabolous insects that develop into adult appendages (legs, antennae, wings, etc.) during metamorphosis from larval to adult form. Sources: GOC:dph, GOC:isa_complete, GOC:jid